{
  "gene_symbol": "SMCR8",
  "gene": "UniProtKB:Q8TEV9",
  "gene_name": "Guanine nucleotide exchange protein SMCR8",
  "term_id": "GO:0032045",
  "term_label": "guanyl-nucleotide exchange factor complex"
}